{
  "gene_name": "Menin",
  "term_label": "transcription cis-regulatory region binding",
  "gene_symbol": "MEN1",
  "gene": "UniProtKB:O00255",
  "term_id": "GO:0000976"
}